nucleosome array spacer activity [GO:0140750] (molecular function) References: PMID:11683384, PMID:16468993 Definition: A histone octamer slider activity that spaces nucleosomes along chromosomal DNA. This activity is involved in assembling chromatin in uniform nucleosome arrays to regulate transcription by RNA polymerases I, II, and III, as well as DNA replication, recombination and repair. Note: In Drosphila, this is mediated by ISWI, in human, by SMARCA5 and in S. cerevisiae by ISW1 and and ISW2. Relationships: is a type of histone octamer slider activity [GO:0140751] Also known as: nucleosome array spacing activity